{
  "gene": "UniProtKB:O14990",
  "term_id": "GO:0004864",
  "term_label": "protein phosphatase inhibitor activity",
  "gene_symbol": "PPP1R2C",
  "gene_name": "Protein phosphatase inhibitor 2 family member C"
}